reductive pentose-phosphate cycle [GO:0019253] (biological process) Relationships: is a type of photosynthesis, dark reaction [GO:0019685]; BFO_0000050 GO:0015977 Also known as: C3 photosynthesis, Calvin cycle Sources: ISBN:0198547684 Definition: The fixation of carbon dioxide (CO2) as glucose in the chloroplasts of C3 plants; uses ATP and NADPH formed in the light reactions of photosynthesis; carbon dioxide reacts with ribulose 1,5-bisphosphate (catalyzed by the function of ribulose-bisphosphate carboxylase) to yield two molecules of 3-phosphoglycerate; these are then phosphorylated by ATP to 1,3-bisphosphateglyceraldehyde which, in turn, is then reduced by NADPH to glyceraldehyde 3-phosphate. The glyceraldehyde 3-phosphate is converted to fructose 5-phosphate and ribulose 5-phosphate by aldolase and other enzymes; the ribulose 5-phosphate is phosphorylated by ATP to ribulose 1,5-bisphosphate. Regulation: regulated by GO:0080152; negatively regulated by GO:0080153 Note: See also the molecular function term 'ribulose-bisphosphate carboxylase activity ; GO:0016984'.